positive regulation of gibberellic acid mediated signaling pathway [GO:0009939] (biological process) Relationships: is a type of regulation of gibberellic acid mediated signaling pathway [GO:0009937]; is a type of positive regulation of signal transduction [GO:0009967]; positively regulates GO:0009740 Sources: GOC:sm Also known as: positive regulation of gibberellic acid mediated signalling, up regulation of gibberellic acid mediated signaling, up-regulation of gibberellic acid mediated signaling, upregulation of gibberellic acid mediated signaling, activation of gibberellic acid mediated signaling, stimulation of gibberellic acid mediated signaling Definition: Any process that activates or increases the frequency, rate or extent of gibberellic acid mediated signaling activity.